ketohexokinase activity [GO:0004454] (molecular function) Also known as: hepatic fructokinase activity, ATP:D-fructose 1-phosphotransferase activity, ketohexokinase (phosphorylating) Sources: EC:2.7.1.3 Relationships: is a type of phosphotransferase activity, alcohol group as acceptor [GO:0016773]; is a type of carbohydrate kinase activity [GO:0019200] Definition: Catalysis of the reaction: ATP + D-fructose = ADP + D-fructose 1-phosphate.